{
  "term_id": "GO:0000149",
  "term_label": "SNARE binding",
  "gene_symbol": "SYT6",
  "gene_name": "Synaptotagmin-6",
  "gene": "UniProtKB:Q5T7P8"
}